{
  "gene": "UniProtKB:P01920",
  "term_label": "MHC class II protein complex binding",
  "gene_symbol": "HLA-DQB1",
  "term_id": "GO:0023026",
  "gene_name": "HLA class II histocompatibility antigen, DQ beta 1 chain"
}